{
  "gene": "UniProtKB:Q9BQ52",
  "term_id": "GO:0042781",
  "term_label": "3'-tRNA processing endoribonuclease activity",
  "gene_name": "Zinc phosphodiesterase ELAC protein 2",
  "gene_symbol": "ELAC2"
}